dorsal motor nucleus of vagus nerve maturation [GO:0035761] (biological process) Relationships: is a type of GO:0071695; is part of dorsal motor nucleus of vagus nerve development [GO:0021744] Definition: A developmental process, independent of morphogenetic (shape) change, that is required for the dorsal motor nucleus of the vagus nerve to attain its fully functional state. Sources: GOC:dgh